positive regulation of neutrophil mediated killing of gram-positive bacterium [GO:0070964] (biological process) Definition: Any process that increases the frequency, rate or extent of the directed killing of a gram-positive bacterium by a neutrophil. Relationships: is a type of regulation of neutrophil mediated killing of gram-positive bacterium [GO:0070952]; is a type of GO:0070962; positively regulates neutrophil-mediated killing of gram-positive bacterium [GO:0070946] Also known as: up regulation of neutrophil mediated killing of gram-positive bacterium, up-regulation of neutrophil mediated killing of gram-positive bacterium, upregulation of neutrophil mediated killing of gram-positive bacterium, activation of neutrophil mediated killing of gram-positive bacterium, stimulation of neutrophil mediated killing of gram-positive bacterium Sources: GOC:add, GOC:mah